{
  "gene": "UniProtKB:Q9P2W6",
  "gene_symbol": "C11orf21",
  "term_id": "UNKNOWN:0002",
  "gene_name": "Uncharacterized protein C11orf21",
  "term_label": "Unknown biological process"
}